{
  "gene_symbol": "TCEA1",
  "gene": "UniProtKB:P23193",
  "term_label": "transcription elongation by RNA polymerase II",
  "gene_name": "Transcription elongation factor A protein 1",
  "term_id": "GO:0006368"
}